{
  "gene_name": "Collagen alpha-1(I) chain",
  "term_label": "Unknown biological process",
  "term_id": "UNKNOWN:0002",
  "gene": "UniProtKB:P02452",
  "gene_symbol": "COL1A1"
}